{
  "term_label": "actin filament binding",
  "gene_symbol": "GAS2L3",
  "term_id": "GO:0051015",
  "gene_name": "GAS2-like protein 3",
  "gene": "UniProtKB:Q86XJ1"
}